{
  "term_label": "heart development",
  "gene_symbol": "PDLIM3",
  "term_id": "GO:0007507",
  "gene_name": "PDZ and LIM domain protein 3",
  "gene": "UniProtKB:Q53GG5"
}